{
  "term_id": "GO:0003730",
  "gene_symbol": "CARHSP1",
  "term_label": "mRNA 3'-UTR binding",
  "gene": "UniProtKB:Q9Y2V2",
  "gene_name": "Calcium-regulated heat-stable protein 1"
}